glycolate transport [GO:1900866] (biological process) Sources: GOC:TermGenie, GOC:pr Subtypes: glycolate transmembrane transport [GO:0097339] Definition: The directed movement of a glycolate into, out of or within a cell, or between cells, by means of some agent such as a transporter or pore. Relationships: is a type of GO:0015718; is a type of organic hydroxy compound transport [GO:0015850]